{
  "term_label": "exocytosis",
  "gene_symbol": "SCAMP3",
  "term_id": "GO:0006887",
  "gene": "UniProtKB:O14828",
  "gene_name": "Secretory carrier-associated membrane protein 3"
}